{
  "term_id": "GO:0005739",
  "gene_name": "Alpha-methylacyl-CoA racemase",
  "gene": "UniProtKB:Q9UHK6",
  "term_label": "mitochondrion",
  "gene_symbol": "AMACR"
}